brainstem development [GO:0003360] (biological process) Definition: The progression of the brainstem from its formation to the mature structure. The brainstem is the part of the brain that connects the brain with the spinal cord. Sources: GOC:dph Relationships: is a type of anatomical structure development [GO:0048856]